{
  "gene_name": "Golgin subfamily A member 6-like protein 24",
  "gene": "UniProtKB:P0DX00",
  "term_id": "UNKNOWN:0003",
  "term_label": "Unknown cellular component",
  "gene_symbol": "GOLGA6L24"
}